transcription by RNA polymerase I [GO:0006360] (biological process) Subtypes: nucleolar large rRNA transcription by RNA polymerase I [GO:0042790] Regulation: regulated by GO:0006356; negatively regulated by negative regulation of transcription by RNA polymerase I [GO:0016479]; positively regulated by positive regulation of transcription by RNA polymerase I [GO:0045943] Relationships: is a type of DNA-templated transcription [GO:0006351] Definition: The synthesis of RNA from a DNA template by RNA polymerase I (RNAP I), originating at an RNAP I promoter. Also known as: transcription from Pol I promoter, transcription from RNA polymerase I promoter, RNA polymerase I transcription factor activity Sources: GOC:jl, GOC:txnOH